{
  "term_id": "GO:0034364",
  "term_label": "high-density lipoprotein particle",
  "gene": "UniProtKB:P11597",
  "gene_name": "Cholesteryl ester transfer protein",
  "gene_symbol": "CETP"
}